regulation of protein localization [GO:0032880] (biological process) Definition: Any process that modulates the frequency, rate or extent of any process in which a protein is transported to, or maintained in, a specific location. Sources: GOC:dph, GOC:mah, GOC:tb Also known as: regulation of cellular protein localisation, regulation of cellular protein localization, regulation of protein localisation Relationships: is a type of regulation of localization [GO:0032879]; regulates intracellular protein localization [GO:0008104] Subtypes: regulation of establishment of protein localization [GO:0070201], regulation of protein localization to lysosome [GO:0150031], regulation of protein localization to cell-cell junction [GO:0150106], regulation of protein localization to nucleus [GO:1900180], regulation of protein localization to cell division site [GO:1901900], regulation of protein localization to spindle pole body [GO:1902363], regulation of protein localization to synapse [GO:1902473], regulation of protein localization to microtubule [GO:1902816], regulation of protein localization to cell tip [GO:1903066], regulation of protein localization to cilium [GO:1903564], negative regulation of protein localization [GO:1903828], positive regulation of protein localization [GO:1903829], GO:1904375, regulation of protein localization to centrosome [GO:1904779], regulation of asymmetric protein localization involved in cell fate determination [GO:1904785], GO:1904814, regulation of protein localization to phagocytic vesicle [GO:1905169], regulation of protein localization to kinetochore [GO:1905340], GO:1905475, GO:1905550, regulation of protein localization to chromatin [GO:1905634], GO:1905666, GO:1905871, regulation of protein localization to cell surface [GO:2000008]